{
  "term_label": "3'-5'-RNA exonuclease activity",
  "gene_name": "Exosome complex exonuclease RRP44",
  "gene_symbol": "DIS3",
  "term_id": "GO:0000175",
  "gene": "UniProtKB:Q9Y2L1"
}